{
  "term_label": "microtubule binding",
  "gene": "UniProtKB:P46821",
  "gene_symbol": "MAP1B",
  "term_id": "GO:0008017",
  "gene_name": "Microtubule-associated protein 1B"
}